{
  "term_id": "GO:0042981",
  "gene_name": "Inactive ubiquitin carboxyl-terminal hydrolase 17-like protein 7",
  "gene": "UniProtKB:P0C7H9",
  "term_label": "regulation of apoptotic process",
  "gene_symbol": "USP17L7"
}